inhibin A complex [GO:0043512] (cellular component) Definition: Heterodimeric hormone composed of an inhibin alpha subunit complexed with an inhibin beta-A subunit. Note: Note that the actions of the inhibin complex are the opposite of those of the activin complex, which is a dimer of an inhibin beta-A and/or inhibin beta-B subunit. See also the cellular component term 'activin complex ; GO:0048180'. Sources: GOC:jl Relationships: is a type of inhibin complex [GO:0043511]